{
  "gene_name": "Zinc finger and BTB domain-containing protein 49",
  "term_label": "regulation of cytokine production",
  "term_id": "GO:0001817",
  "gene_symbol": "ZBTB49",
  "gene": "UniProtKB:Q6ZSB9"
}